{
  "gene": "UniProtKB:Q8TDB8",
  "gene_symbol": "SLC2A14",
  "term_label": "plasma membrane",
  "term_id": "GO:0005886",
  "gene_name": "Solute carrier family 2, facilitated glucose transporter member 14"
}